{
  "gene": "UniProtKB:Q8WVM8",
  "gene_name": "Sec1 family domain-containing protein 1",
  "gene_symbol": "SCFD1",
  "term_label": "endoplasmic reticulum to Golgi vesicle-mediated transport",
  "term_id": "GO:0006888"
}